{
  "term_id": "GO:0010008",
  "gene_symbol": "APPL2",
  "term_label": "endosome membrane",
  "gene": "UniProtKB:Q8NEU8",
  "gene_name": "DCC-interacting protein 13-beta"
}